{
  "term_label": "heterotrimeric G-protein complex",
  "gene_name": "Guanine nucleotide-binding protein subunit beta-5",
  "gene": "UniProtKB:O14775",
  "gene_symbol": "GNB5",
  "term_id": "GO:0005834"
}